{
  "term_label": "Unknown cellular component",
  "gene_symbol": "Q8N976",
  "gene_name": "Putative uncharacterized protein FLJ38264",
  "term_id": "UNKNOWN:0003",
  "gene": "UniProtKB:Q8N976"
}